{
  "gene_symbol": "OR6K2",
  "gene": "UniProtKB:Q8NGY2",
  "gene_name": "Olfactory receptor 6K2",
  "term_id": "GO:0050911",
  "term_label": "detection of chemical stimulus involved in sensory perception of smell"
}